{
  "gene": "UniProtKB:A0PJW8",
  "term_id": "UNKNOWN:0003",
  "gene_symbol": "DAPL1",
  "gene_name": "Death-associated protein-like 1",
  "term_label": "Unknown cellular component"
}